{
  "term_label": "nervous system development",
  "gene": "UniProtKB:Q8WYK1",
  "gene_symbol": "CNTNAP5",
  "term_id": "GO:0007399",
  "gene_name": "Contactin-associated protein-like 5"
}